neurotransmitter receptor transport postsynaptic membrane to endosome [GO:0098968] (biological process) Definition: Vesicle-mediated transport of a neurotransmitter receptor complex from the postsynaptic membrane to the postsynaptic early endosome. Relationships: is a type of vesicle-mediated transport [GO:0016192]; is a type of receptor localization to synapse [GO:0097120] Sources: GOC:dos